extrinsic component of postsynaptic specialization membrane [GO:0098892] (cellular component) Relationships: is a type of extrinsic component of postsynaptic membrane [GO:0098890]; is part of GO:0099634 Subtypes: extrinsic component of postsynaptic density membrane [GO:0099147] Sources: GOC:autophagy, GOC:mf Definition: The component of the postsynaptic specialization membrane consisting of gene products and protein complexes that are loosely bound to one of its surfaces, but not integrated into the hydrophobic region.